{
  "term_label": "plasma membrane",
  "gene_name": "T cell receptor beta variable 7-2",
  "gene_symbol": "TRBV7-2",
  "term_id": "GO:0005886",
  "gene": "UniProtKB:A0A1B0GXF2"
}